{
  "term_label": "endoplasmic reticulum to Golgi vesicle-mediated transport",
  "gene_name": "B-cell receptor-associated protein 29",
  "term_id": "GO:0006888",
  "gene_symbol": "BCAP29",
  "gene": "UniProtKB:Q9UHQ4"
}